{
  "term_label": "phosphatidylinositol-3,5-bisphosphate phosphatase activity",
  "gene_name": "Myotubularin-related protein 7",
  "term_id": "GO:0106018",
  "gene_symbol": "MTMR7",
  "gene": "UniProtKB:Q9Y216"
}